maintenance of membrane potential in photoreceptor cell by rhodopsin mediated signaling [GO:0016058] (biological process) Also known as: maintenance of rhodopsin mediated signalling, maintenance of rhodopsin mediated signaling Definition: Maintenance of the excited state of a photoreceptor cell to produce a steady-state current as a result of signals generated by rhodopsin activation by a photon. Relationships: is a type of regulation of membrane potential in photoreceptor cell [GO:0016057] Sources: GOC:dph, GOC:hb, GOC:tb